{
  "gene_symbol": "MAPKAPK5",
  "gene_name": "MAP kinase-activated protein kinase 5",
  "term_id": "GO:0032007",
  "gene": "UniProtKB:Q8IW41",
  "term_label": "negative regulation of TOR signaling"
}